{
  "term_id": "UNKNOWN:0001",
  "gene_symbol": "COCH",
  "gene": "UniProtKB:O43405",
  "term_label": "Unknown molecular function",
  "gene_name": "Cochlin"
}